maleylpyruvate isomerase activity [GO:0050077] (molecular function) Definition: Catalysis of the reaction: 3-maleylpyruvate = 3-fumarylpyruvate. Relationships: is a type of cis-trans isomerase activity [GO:0016859] Sources: EC:5.2.1.4, MetaCyc:MALEYLPYRUVATE-ISOMERASE-RXN Also known as: 3-maleylpyruvate cis-trans-isomerase activity